natural killer cell proliferation involved in immune response [GO:0002324] (biological process) Definition: The expansion of a natural killer cell population by cell division as part of an immune response. Relationships: is a type of natural killer cell proliferation [GO:0001787]; is_a lymphocyte activation involved in immune response [GO:0002285] Regulation: regulated by regulation of natural killer cell proliferation involved in immune response [GO:0032820]; negatively regulated by negative regulation of natural killer cell proliferation involved in immune response [GO:0032821]; positively regulated by positive regulation of natural killer cell proliferation involved in immune response [GO:0032822] References: PMID:15032583 Sources: GOC:add Also known as: NK cell proliferation during immune response, natural killer cell proliferation during immune response